{
  "gene": "UniProtKB:Q96SB4",
  "term_label": "nucleus",
  "gene_name": "SRSF protein kinase 1",
  "gene_symbol": "SRPK1",
  "term_id": "GO:0005634"
}